maturation of SSU-rRNA from tetracistronic rRNA transcript (SSU-rRNA, LSU-rRNA, 4.5S-rRNA, 5S-rRNA) [GO:0000489] (biological process) Relationships: is a type of maturation of SSU-rRNA [GO:0030490] Sources: GOC:curators Definition: Any process involved in the maturation of a precursor Small SubUnit (SSU) ribosomal RNA (rRNA) molecule into a mature SSU-rRNA molecule from the pre-rRNA molecule originally produced as a tetracistronic rRNA transcript that contains the Small Subunit (SSU) rRNA, Large Subunit (LSU) the 4.5S rRNA, and the 5S rRNA in that order from 5' to 3' along the primary transcript.